{
  "term_id": "GO:0005634",
  "gene_symbol": "RBP7",
  "gene": "UniProtKB:Q96R05",
  "term_label": "nucleus",
  "gene_name": "Retinoid-binding protein 7"
}